{
  "term_label": "endoplasmic reticulum tubular network",
  "gene_symbol": "ZFYVE27",
  "gene_name": "Protrudin",
  "term_id": "GO:0071782",
  "gene": "UniProtKB:Q5T4F4"
}